methylglutaconyl-CoA hydratase activity [GO:0004490] (molecular function) Sources: EC:4.2.1.18, RHEA:21536 Relationships: is a type of hydro-lyase activity [GO:0016836] Definition: Catalysis of the reaction: (S)-3-hydroxy-3-methylglutaryl-CoA = trans-3-methylglutaconyl-CoA + H2O. Also known as: (S)-3-hydroxy-3-methylglutaryl-CoA hydro-lyase (trans-3-methylglutaconyl-CoA-forming), (S)-3-hydroxy-3-methylglutaryl-CoA hydro-lyase activity, 3-methylglutaconyl CoA hydratase activity, methylglutaconase activity, methylglutaconyl coenzyme A hydratase activity